regulation of endothelial cell chemotaxis to fibroblast growth factor [GO:2000544] (biological process) Sources: GOC:obol Definition: Any process that modulates the frequency, rate or extent of endothelial cell chemotaxis to fibroblast growth factor. Subtypes: negative regulation of endothelial cell chemotaxis to fibroblast growth factor [GO:2000545], positive regulation of endothelial cell chemotaxis to fibroblast growth factor [GO:2000546] Relationships: is a type of GO:1904847; is a type of GO:2001026; RO_0002211 GO:0035768